{
  "gene_name": "Nonsense-mediated mRNA decay factor SMG5",
  "term_id": "GO:0000184",
  "gene_symbol": "SMG5",
  "gene": "UniProtKB:Q9UPR3",
  "term_label": "nuclear-transcribed mRNA catabolic process, nonsense-mediated decay"
}